(R)-dehydropantoate dehydrogenase activity [GO:0047509] (molecular function) Definition: Catalysis of the reaction: (R)-4-dehydropantoate + H2O + NAD+ = (R)-3,3-dimethylmalate + 2 H+ + NADH. Also known as: (R)-4-dehydropantoate:NAD+ 4-oxidoreductase activity, D-2-hydroxy-3,3-dimethyl-3-formylpropionate:diphosphopyridine nucleotide (DPN+) oxidoreductase activity, D-aldopantoate dehydrogenase activity Relationships: is_a oxidoreductase activity, acting on the aldehyde or oxo group of donors, NAD or NADP as acceptor [GO:0016620] Sources: EC:1.2.1.33, RHEA:19349